{
  "term_label": "plasma membrane",
  "term_id": "GO:0005886",
  "gene_symbol": "CNTN5",
  "gene_name": "Contactin-5",
  "gene": "UniProtKB:O94779"
}